{
  "term_id": "GO:1900118",
  "gene_name": "Humanin-like 2",
  "gene_symbol": "MTRNR2L2",
  "gene": "UniProtKB:P0CJ69",
  "term_label": "negative regulation of execution phase of apoptosis"
}